ureteric bud morphogenesis [GO:0060675] (biological process) Relationships: is a type of GO:0072171; is part of GO:0001657 Sources: GOC:dph, GOC:mtg_kidney_jan10 Definition: The process in which the ureteric bud is generated and organized.